{
  "gene": "UniProtKB:C9JXX5",
  "gene_symbol": "FREY1",
  "term_id": "GO:0035036",
  "term_label": "sperm-egg recognition",
  "gene_name": "Protein Frey 1"
}